positive regulation of renal sodium excretion [GO:0035815] (biological process) Sources: GOC:mtg_25march11, GOC:yaf Subtypes: positive regulation of renal sodium excretion by pressure natriuresis [GO:0035819] Relationships: is a type of GO:0035813; is a type of positive regulation of secretion [GO:0051047]; is a type of GO:0051240; positively regulates renal sodium excretion [GO:0035812] Note: The amount of sodium excreted in urine over a unit of time can be increased by increasing the volume of urine produced (diuresis) and/or by increasing the concentration of sodium in the urine. Also known as: natriuresis Definition: Any process that increases the amount of sodium excreted in urine over a unit of time.